{
  "gene_symbol": "FASLG",
  "term_id": "GO:0043123",
  "term_label": "positive regulation of canonical NF-kappaB signal transduction",
  "gene": "UniProtKB:P48023",
  "gene_name": "Tumor necrosis factor ligand superfamily member 6"
}